{
  "gene": "UniProtKB:P51665",
  "gene_symbol": "PSMD7",
  "term_label": "Unknown molecular function",
  "term_id": "UNKNOWN:0001",
  "gene_name": "26S proteasome non-ATPase regulatory subunit 7"
}